cellular response to alcohol [GO:0097306] (biological process) Relationships: is_a response to alcohol [GO:0097305]; is a type of GO:1901701 Sources: GOC:pr Subtypes: cellular response to abscisic acid stimulus [GO:0071215], GO:0071301, cellular response to ethanol [GO:0071361], cellular response to prostaglandin E stimulus [GO:0071380], cellular response to corticosterone stimulus [GO:0071386], cellular response to cortisol stimulus [GO:0071387], GO:0071388, cellular response to ecdysone [GO:0071390], GO:0071397, GO:0071405, GO:0071409, cellular response to indole-3-methanol [GO:0071681], cellular response to prostaglandin D stimulus [GO:0071799], GO:0072705, cellular response to tetracycline [GO:0072746], cellular response to rapamycin [GO:0072752], cellular response to camptothecin [GO:0072757], GO:0097308, cellular response to ergosterol [GO:1901625], cellular response to dehydroepiandrosterone [GO:1903495], GO:1903497, GO:1904045, cellular response to forskolin [GO:1904322], cellular response to diphenidol [GO:1904561], cellular response to phorbol 13-acetate 12-myristate [GO:1904628], GO:1905093, cellular response to haloperidol [GO:1905120] Regulation: regulated by regulation of cellular response to alcohol [GO:1905957]; negatively regulated by GO:1905958; positively regulated by positive regulation of cellular response to alcohol [GO:1905959] Definition: Any process that results in a change in state or activity of a cell (in terms of movement, secretion, enzyme production, gene expression, etc.) as a result of an alcohol stimulus.